vesicle targeting [GO:0006903] (biological process) Definition: The process in which vesicles are directed to specific destination membranes. Targeting involves coordinated interactions among cytoskeletal elements (microtubules or actin filaments), motor proteins, molecules at the vesicle membrane and target membrane surfaces, and vesicle cargo. References: PMID:17335816 Sources: GOC:mah Relationships: is a type of cellular process [GO:0009987]; is part of vesicle-mediated transport [GO:0016192]; is part of establishment of vesicle localization [GO:0051650] Subtypes: synaptic vesicle targeting [GO:0016080], vesicle targeting to fusome [GO:0045479], vesicle targeting, to, from or within Golgi [GO:0048199], vesicle targeting, plasma membrane to endosome [GO:0048201], contractile vacuole tethering involved in discharge [GO:0140025]